{
  "gene": "UniProtKB:Q9NQ89",
  "gene_symbol": "C12orf4",
  "gene_name": "Protein C12orf4",
  "term_label": "Unknown molecular function",
  "term_id": "UNKNOWN:0001"
}